{
  "gene": "UniProtKB:Q8N6F1",
  "term_id": "GO:0005886",
  "gene_name": "Claudin-19",
  "gene_symbol": "CLDN19",
  "term_label": "plasma membrane"
}